{
  "term_id": "UNKNOWN:0001",
  "gene": "UniProtKB:Q04760",
  "term_label": "Unknown molecular function",
  "gene_name": "Lactoylglutathione lyase",
  "gene_symbol": "GLO1"
}